{
  "term_id": "GO:0098839",
  "term_label": "postsynaptic density membrane",
  "gene_name": "Germ cell-specific gene 1-like protein",
  "gene_symbol": "GSG1L",
  "gene": "UniProtKB:Q6UXU4"
}